negative regulation of aortic smooth muscle cell differentiation [GO:1904830] (biological process) Definition: Any process that stops, prevents or reduces the frequency, rate or extent of aortic smooth muscle cell differentiation. References: PMID:22034194 Sources: GOC:BHF, GOC:BHF_miRNA, GOC:TermGenie, GOC:rph, GO_REF:0000058 Also known as: down regulation of aortic smooth muscle cell differentiation, down-regulation of aortic smooth muscle cell differentiation, downregulation of aortic smooth muscle cell differentiation, inhibition of aortic smooth muscle cell differentiation Relationships: is a type of regulation of aortic smooth muscle cell differentiation [GO:1904829]; is a type of negative regulation of vascular associated smooth muscle cell differentiation [GO:1905064]; negatively regulates aortic smooth muscle cell differentiation [GO:0035887]